{
  "gene": "UniProtKB:O14646",
  "gene_name": "Chromodomain-helicase-DNA-binding protein 1",
  "term_label": "ATP hydrolysis activity",
  "term_id": "GO:0016887",
  "gene_symbol": "CHD1"
}